{
  "gene_symbol": "NPY2R",
  "gene": "UniProtKB:P49146",
  "term_id": "GO:0007218",
  "gene_name": "Neuropeptide Y receptor type 2",
  "term_label": "neuropeptide signaling pathway"
}